regulation of amine transport [GO:0051952] (biological process) Relationships: is a type of regulation of transport [GO:0051049]; regulates amine transport [GO:0015837] Sources: GOC:ai Definition: Any process that modulates the frequency, rate or extent of the directed movement of amines into, out of or within a cell, or between cells, by means of some agent such as a transporter or pore. Subtypes: regulation of acetylcholine secretion, neurotransmission [GO:0014056], GO:0050433, regulation of acetylcholine uptake [GO:0051631], regulation of catecholamine uptake involved in synaptic transmission [GO:0051940], negative regulation of amine transport [GO:0051953], positive regulation of amine transport [GO:0051954], regulation of amino acid transport [GO:0051955]